phosphoribosylglycinamide formyltransferase activity [GO:0004644] (molecular function) Definition: Catalysis of the reaction: 10-formyltetrahydrofolate + N1-(5-phospho-D-ribosyl)glycinamide = tetrahydrofolate + N2-formyl-N1-(5-phospho-D-ribosyl)glycinamide. Relationships: is a type of hydroxymethyl-, formyl- and related transferase activity [GO:0016742] Sources: EC:2.1.2.2 Also known as: 10-formyltetrahydrofolate:5'-phosphoribosylglycinamide N-formyltransferase activity, 2-amino-N-ribosylacetamide 5'-phosphate transformylase activity, 5'-phosphoribosylglycinamide transformylase activity, 5,10-methenyltetrahydrofolate:2-amino-N-ribosylacetamide ribonucleotide transformylase activity, GAR TFase activity, GAR formyltransferase activity, GAR transformylase activity, GART activity, glycinamide ribonucleotide transformylase activity